{
  "gene_symbol": "ANTXRL",
  "gene": "UniProtKB:A6NF34",
  "term_label": "plasma membrane",
  "gene_name": "Anthrax toxin receptor-like",
  "term_id": "GO:0005886"
}